{
  "gene_symbol": "ANTXR1",
  "term_label": "Unknown biological process",
  "gene": "UniProtKB:Q9H6X2",
  "gene_name": "Anthrax toxin receptor 1",
  "term_id": "UNKNOWN:0002"
}